{
  "term_label": "Unknown biological process",
  "gene": "UniProtKB:A2RUU4",
  "gene_symbol": "CLPSL1",
  "term_id": "UNKNOWN:0002",
  "gene_name": "Colipase-like protein 1"
}